{
  "term_label": "mitochondrial inner membrane",
  "gene_symbol": "UQCC4",
  "gene": "UniProtKB:Q4G0I0",
  "term_id": "GO:0005743",
  "gene_name": "Ubiquinol-cytochrome-c reductase complex assembly factor 4"
}